cardiac jelly development [GO:1905072] (biological process) Relationships: is a type of tissue development [GO:0009888]; BFO_0000050 GO:0007507 Also known as: heart cardiac jelly development References: PMID:10645959, PMID:16314491, PMID:19703439 Sources: GOC:BHF, GOC:TermGenie, GOC:rl, GO_REF:0000094 Definition: The process whose specific outcome is the progression of cardiac jelly over time, from its formation to the mature structure. The cardiac jelly is an acellular gelatinous matrix secreted by the myocardium and plays a central role in the septation of the heart.